{
  "term_id": "GO:0004806",
  "gene_symbol": "PNPLA5",
  "gene_name": "Patatin-like phospholipase domain-containing protein 5",
  "gene": "UniProtKB:Q7Z6Z6",
  "term_label": "triacylglycerol lipase activity"
}